{
  "term_id": "UNKNOWN:0001",
  "gene": "UniProtKB:Q8N690",
  "term_label": "Unknown molecular function",
  "gene_symbol": "DEFB119",
  "gene_name": "Beta-defensin 119"
}